positive regulation of ascospore formation [GO:0075296] (BP) Definition: Any process that activates, maintains or increases the frequency, rate or extent of ascospore formation, a process in which a sexual spore, named ascospore, from Ascomycete fungi was produced inside an ascus. Sources: GOC:pamgo_curators Relationships: is a type of positive regulation of cell development [GO:0010720]; is a type of regulation of ascospore formation [GO:0034307]; is a type of positive regulation of sexual sporulation resulting in formation of a cellular spore [GO:0043941]; is a type of GO:0090068; positively regulates ascospore formation [GO:0030437] Subtypes: positive regulation of ascospore-type prospore membrane formation [GO:1903024]